{
  "term_id": "GO:0042923",
  "term_label": "neuropeptide binding",
  "gene": "UniProtKB:P32745",
  "gene_symbol": "SSTR3",
  "gene_name": "Somatostatin receptor type 3"
}